nasal suture morphogenesis [GO:0097097] (biological process) Sources: GOC:pr, GOC:sl, Wikipedia:Cranial_sutures, Wikipedia:Head_and_neck_anatomy#Musculoskeletal_system Relationships: is a type of facial suture morphogenesis [GO:0097096] Also known as: internasal suture morphogenesis Definition: The process in which the nasal suture is generated and organized.